negative regulation of SNARE complex assembly [GO:0035544] (biological process) Sources: GOC:rb Definition: Any process that decreases the frequency, rate or extent of assembly of the SNARE complex. The SNARE complex is a protein complex involved in membrane fusion; a stable ternary complex consisting of a four-helix bundle, usually formed from one R-SNARE and three Q-SNAREs with an ionic layer sandwiched between hydrophobic layers. Relationships: is a type of negative regulation of protein-containing complex assembly [GO:0031333]; is a type of GO:0031339; is a type of regulation of SNARE complex assembly [GO:0035542]; negatively regulates SNARE complex assembly [GO:0035493]